fructose 5-dehydrogenase activity [GO:0047904] (molecular function) Definition: Catalysis of the reaction: a ubiquinone + keto-D-fructose = 5-dehydro-D-fructose + a ubiquinol. Also known as: D-fructose dehydrogenase activity Sources: RHEA:22304 Relationships: is a type of oxidoreductase activity, acting on the CH-OH group of donors, quinone or similar compound as acceptor [GO:0016901]